response to cobalt ion [GO:0032025] (biological process) Relationships: is a type of response to metal ion [GO:0010038] Definition: Any process that results in a change in state or activity of a cell or an organism (in terms of movement, secretion, enzyme production, gene expression, etc.) as a result of a cobalt ion (Co2+) stimulus. Sources: GOC:mah Subtypes: cellular response to cobalt ion [GO:0071279]